endoplasmic reticulum localization [GO:0051643] (biological process) Definition: Any process in which endoplasmic reticulum is transported to, and/or maintained in, a specific location within the cell. Sources: GOC:ai Also known as: ER localization, endoplasmic reticulum localisation, establishment and maintenance of ER localization Relationships: is a type of organelle localization [GO:0051640]; is part of endoplasmic reticulum organization [GO:0007029] Subtypes: maintenance of ER location [GO:0051685], establishment of ER localization [GO:0051686], GO:0061817